{
  "gene_symbol": "DACH1",
  "gene": "UniProtKB:Q9UI36",
  "term_label": "DNA-binding transcription factor activity, RNA polymerase II-specific",
  "gene_name": "Dachshund homolog 1",
  "term_id": "GO:0000981"
}